RNA endonuclease activity producing 3'-phosphomonoesters, hydrolytic mechanism [GO:0016892] (molecular function) Subtypes: ribonuclease F activity [GO:0033900], ribonuclease V activity [GO:0033901] Sources: GOC:ai Definition: Catalysis of the hydrolysis of ester linkages within ribonucleic acids by creating internal breaks to yield 3'-phosphomonoesters. Also known as: endoribonuclease activity, producing 3'-phosphomonoesters, endoribonuclease activity, producing other than 5'-phosphomonoesters Relationships: is a type of GO:0004521; is a type of hydrolase activity, acting on ester bonds [GO:0016788]